basal dendrite [GO:0097441] (cellular component) Relationships: is a type of GO:0030425 Subtypes: GO:0150016, basal proximal dendrite [GO:0150017] Definition: A dendrite that emerges near the basal pole of a neuron. In bipolar neurons, basal dendrites are either on the same side of the soma as the axon, or project toward the axon. References: PMID:17046728, PMID:22683681 Sources: GOC:aruk, GOC:bc, NIF_Subcellular:sao1079900774 Also known as: basilar dendrite